{
  "gene_symbol": "ICAM5",
  "gene": "UniProtKB:Q9UMF0",
  "term_id": "GO:0005178",
  "term_label": "integrin binding",
  "gene_name": "Intercellular adhesion molecule 5"
}